{
  "term_label": "mRNA binding",
  "term_id": "GO:0003729",
  "gene_name": "ATP-dependent RNA helicase DDX50",
  "gene": "UniProtKB:Q9BQ39",
  "gene_symbol": "DDX50"
}